{
  "gene": "UniProtKB:Q5JNZ5",
  "term_id": "GO:0003729",
  "gene_symbol": "RPS26P11",
  "term_label": "mRNA binding",
  "gene_name": "Putative ribosomal protein eS26-like"
}